{
  "gene_name": "Peroxiredoxin-6",
  "gene": "UniProtKB:P30041",
  "term_id": "GO:0045454",
  "gene_symbol": "PRDX6",
  "term_label": "cell redox homeostasis"
}